{
  "term_id": "GO:0016538",
  "gene_name": "Cyclin-L1",
  "gene_symbol": "CCNL1",
  "term_label": "cyclin-dependent protein serine/threonine kinase regulator activity",
  "gene": "UniProtKB:Q9UK58"
}